{
  "gene_name": "ATP-dependent RNA helicase DHX33",
  "term_id": "GO:0045943",
  "gene_symbol": "DHX33",
  "term_label": "positive regulation of transcription by RNA polymerase I",
  "gene": "UniProtKB:Q9H6R0"
}